photosynthesis, light harvesting in photosystem II [GO:0009769] (biological process) Relationships: is a type of photosynthesis, light harvesting [GO:0009765] Definition: After a photon of light is absorbed by one of the many chlorophyll molecules, in one of the light-harvesting complexes of an antenna on photosystem II, some of the absorbed energy is transferred to the pair of chlorophyll molecules in the reaction center. Sources: GOC:jid, ISBN:0716731363, ISBN:0816017360